Golgi cis cisterna membrane [GO:1990674] (cellular component) Relationships: is a type of GO:0032580; is part of Golgi cis cisterna [GO:0000137] References: PMID:16038056, PMID:24119662 Sources: GOC:bhm Definition: The lipid bilayer surrounding any of the thin, flattened compartments that form the cis portion of the Golgi complex. Also known as: Golgi apparatus cis cisterna membrane, cis-Golgi cisterna membrane